{
  "gene_name": "Coiled-coil domain-containing protein 86",
  "gene_symbol": "CCDC86",
  "term_id": "UNKNOWN:0001",
  "term_label": "Unknown molecular function",
  "gene": "UniProtKB:Q9H6F5"
}